{
  "gene_symbol": "TMEM236",
  "gene": "UniProtKB:Q5W0B7",
  "term_id": "UNKNOWN:0002",
  "term_label": "Unknown biological process",
  "gene_name": "Transmembrane protein 236"
}